{
  "term_id": "GO:0055085",
  "gene": "UniProtKB:Q03518",
  "term_label": "transmembrane transport",
  "gene_symbol": "TAP1",
  "gene_name": "Antigen peptide transporter 1"
}